{
  "gene": "UniProtKB:Q86SE8",
  "term_id": "GO:0006338",
  "gene_symbol": "NPM2",
  "gene_name": "Nucleoplasmin-2",
  "term_label": "chromatin remodeling"
}